{
  "gene_symbol": "SETMAR",
  "term_label": "DNA double-strand break processing",
  "term_id": "GO:0000729",
  "gene": "UniProtKB:Q53H47",
  "gene_name": "Histone-lysine N-methyltransferase SETMAR"
}